negative regulation of alcohol catabolic process [GO:1900420] (biological process) Definition: Any process that stops, prevents or reduces the frequency, rate or extent of  alcohol catabolic process within a cell. Sources: GOC:TermGenie Also known as: down regulation of cellular alcohol catabolic process, down-regulation of cellular alcohol catabolic process, downregulation of cellular alcohol catabolic process, inhibition of cellular alcohol catabolic process Relationships: is a type of negative regulation of catabolic process [GO:0009895]; is a type of negative regulation of small molecule metabolic process [GO:0062014]; is a type of regulation of alcohol catabolic process [GO:1900419]; negatively regulates GO:0046164